plasma lipoprotein particle assembly [GO:0034377] (biological process) Subtypes: GO:0034378, GO:0034379, GO:0034380 Relationships: is a type of protein-lipid complex assembly [GO:0065005]; is a type of GO:0071827; BFO_0000050 regulation of plasma lipoprotein particle levels [GO:0097006] Definition: The non-covalent aggregation and arrangement of proteins and lipids to form a plasma lipoprotein particle. Sources: GOC:BHF, GOC:mah